calcium-independent cell-matrix adhesion [GO:0007161] (biological process) Definition: The binding of a cell to the extracellular matrix via adhesion molecules that do not require the presence of calcium for the interaction. Sources: GOC:hb Also known as: calcium-independent cell adhesion molecule activity Relationships: is a type of GO:0007160